{
  "term_id": "GO:1905030",
  "gene_symbol": "KCND2",
  "gene_name": "Potassium voltage-gated channel subfamily D member 2",
  "term_label": "voltage-gated monoatomic ion channel activity involved in regulation of postsynaptic membrane potential",
  "gene": "UniProtKB:Q9NZV8"
}